dendritic spine head [GO:0044327] (cellular component) Sources: GOC:BHF, GOC:nln, GOC:rl Also known as: spine head Relationships: is_a cellular anatomical structure [GO:0110165]; is part of dendritic spine [GO:0043197]; has part postsynaptic density [GO:0014069] Definition: Distal part of the dendritic spine, that carries the post-synaptic density.